{
  "term_label": "extracellular matrix",
  "term_id": "GO:0031012",
  "gene": "UniProtKB:P12110",
  "gene_symbol": "COL6A2",
  "gene_name": "Collagen alpha-2(VI) chain"
}